guanosine binding [GO:1905108] (molecular function) References: PMID:26007660 Sources: GOC:TermGenie, GO_REF:0000067 Definition: Binding to guanosine. Relationships: is a type of purine ribonucleoside binding [GO:0032550]